{
  "term_id": "GO:0007166",
  "gene_symbol": "MILR1",
  "gene_name": "Allergin-1",
  "gene": "UniProtKB:Q7Z6M3",
  "term_label": "cell surface receptor signaling pathway"
}